cardiac left atrium formation [GO:0003216] (biological process) Definition: The developmental process pertaining to the initial formation of a left cardiac atrium from unspecified parts. Relationships: is_a cardiac atrium formation [GO:0003210]; is part of GO:0003212 Sources: GOC:mtg_heart